{
  "term_label": "Unknown biological process",
  "gene_symbol": "CST1",
  "gene_name": "Cystatin-SN",
  "term_id": "UNKNOWN:0002",
  "gene": "UniProtKB:P01037"
}